{
  "term_id": "GO:0045087",
  "term_label": "innate immune response",
  "gene_name": "Interferon lambda-4",
  "gene_symbol": "IFNL4",
  "gene": "UniProtKB:K9M1U5"
}